{
  "term_label": "odorant binding",
  "gene_symbol": "OR13A1",
  "term_id": "GO:0005549",
  "gene": "UniProtKB:Q8NGR1",
  "gene_name": "Olfactory receptor 13A1"
}